{
  "term_label": "Unknown biological process",
  "gene": "UniProtKB:A0A087WZK3",
  "term_id": "UNKNOWN:0002",
  "gene_name": "KRAB domain-containing protein (Fragment)",
  "gene_symbol": "LOC344065"
}